{
  "gene_name": "Paralemmin-1",
  "term_label": "postsynapse",
  "term_id": "GO:0098794",
  "gene_symbol": "PALM",
  "gene": "UniProtKB:O75781"
}